{
  "gene_symbol": "CIB1",
  "term_id": "GO:0005509",
  "gene_name": "Calcium and integrin-binding protein 1",
  "term_label": "calcium ion binding",
  "gene": "UniProtKB:Q99828"
}